{
  "term_label": "olfactory receptor activity",
  "gene_symbol": "OR5M1",
  "gene": "UniProtKB:Q8NGP8",
  "term_id": "GO:0004984",
  "gene_name": "Olfactory receptor 5M1"
}